beta-heterochromatin [GO:0005722] (cellular component) Relationships: is a type of pericentric heterochromatin [GO:0005721]; is part of GO:0005701 References: PMID:11404334, PMID:8878678 Definition: A diffusely banded region of heterochromatin located between euchromatin and alpha-heterochromatin in the polytene chromosome chromocenter; normally replicated during polytenization.